endoplasmic reticulum-lipid droplet tether activity [GO:0170007] (molecular function) Definition: The binding activity of a molecule that brings together a lipid droplet with an endoplasmic reticulum membrane, via membrane lipid binding, to establish membrane contact sites and mediate exchange and communication. Relationships: is a type of protein-membrane adaptor activity [GO:0043495] References: PMID:35389430